{
  "term_id": "GO:0004815",
  "term_label": "aspartate-tRNA ligase activity",
  "gene_name": "Aspartate--tRNA ligase, mitochondrial",
  "gene": "UniProtKB:Q6PI48",
  "gene_symbol": "DARS2"
}